{
  "term_id": "UNKNOWN:0003",
  "term_label": "Unknown cellular component",
  "gene_symbol": "TCF24",
  "gene_name": "Transcription factor 24",
  "gene": "UniProtKB:Q7RTU0"
}